{
  "gene": "UniProtKB:Q96NA8",
  "term_label": "SNAP receptor activity",
  "gene_symbol": "TSNARE1",
  "term_id": "GO:0005484",
  "gene_name": "t-SNARE domain-containing protein 1"
}